negative regulation of tight junction disassembly [GO:1905074] (biological process) References: PMID:18718461 Sources: GOC:BHF, GOC:TermGenie, GOC:rl, GO_REF:0000058 Also known as: down regulation of occluding cell junction disassembly, down regulation of tight junction disassembly, down-regulation of occluding cell junction disassembly, down-regulation of tight junction disassembly, downregulation of occluding cell junction disassembly, downregulation of occluding junction disassembly, downregulation of tight junction disassembly, negative regulation of occluding cell junction disassembly, inhibition of occluding cell junction disassembly, inhibition of occluding junction disassembly, inhibition of tight junction disassembly Relationships: is a type of negative regulation of cellular component organization [GO:0051129]; is a type of GO:1905073; negatively regulates tight junction disassembly [GO:1905071] Definition: Any process that stops, prevents or reduces the frequency, rate or extent of tight junction disassembly.